regulation of DNA binding [GO:0051101] (biological process) Definition: Any process that modulates the frequency, rate or extent of DNA binding. DNA binding is any process in which a gene product interacts selectively with DNA (deoxyribonucleic acid). Relationships: is a type of regulation of binding [GO:0051098]; regulates DNA binding [GO:0003677] Subtypes: GO:0043388, GO:0043392, regulation of transcription regulatory region DNA binding [GO:2000677] Sources: GOC:ai, GOC:dph, GOC:tb